{
  "gene_name": "Protocadherin gamma-A5",
  "gene": "UniProtKB:Q9Y5G8",
  "term_label": "plasma membrane",
  "gene_symbol": "PCDHGA5",
  "term_id": "GO:0005886"
}